3-chlorobenzoate-3,4-oxygenase activity [GO:0102045] (molecular function) Relationships: is a type of oxidoreductase activity, acting on paired donors, with incorporation or reduction of molecular oxygen, NAD(P)H as one donor, and incorporation of two atoms of oxygen into one donor [GO:0016708] References: PMID:8285670 Sources: GOC:pz Definition: Catalysis of the reaction: 3-chlorobenzoate + O2 + a reduced electron acceptor = 3-chlorobenzoate-cis-3,4-diol + an oxidized electron acceptor.